{
  "term_label": "Unknown cellular component",
  "gene_name": "Otospiralin",
  "term_id": "UNKNOWN:0003",
  "gene": "UniProtKB:Q8NHW6",
  "gene_symbol": "OTOS"
}